{
  "gene_name": "G antigen 12F",
  "gene_symbol": "GAGE12F",
  "term_label": "Unknown molecular function",
  "term_id": "UNKNOWN:0001",
  "gene": "UniProtKB:P0CL80"
}